{
  "gene": "UniProtKB:Q9NQT8",
  "term_label": "microtubule binding",
  "gene_symbol": "KIF13B",
  "gene_name": "Kinesin-like protein KIF13B",
  "term_id": "GO:0008017"
}